{
  "gene_name": "Cell surface glycoprotein MUC18",
  "gene_symbol": "MCAM",
  "term_id": "GO:0005886",
  "gene": "UniProtKB:P43121",
  "term_label": "plasma membrane"
}